{
  "gene": "UniProtKB:P52657",
  "term_label": "RNA polymerase II preinitiation complex assembly",
  "term_id": "GO:0051123",
  "gene_name": "Transcription initiation factor IIA subunit 2",
  "gene_symbol": "GTF2A2"
}